{
  "term_id": "GO:0005737",
  "gene": "UniProtKB:Q9UHN1",
  "term_label": "cytoplasm",
  "gene_symbol": "POLG2",
  "gene_name": "DNA polymerase subunit gamma-2, mitochondrial"
}